pyrimidine ribonucleotide binding [GO:0032557] (molecular function) Subtypes: UTP binding [GO:0002134], GO:0002135 Definition: Binding to a pyrimidine ribonucleotide, any compound consisting of a pyrimidine ribonucleoside that is esterified with (ortho)phosphate or an oligophosphate at any hydroxyl group on the ribose moiety. Sources: GOC:mah Relationships: is a type of pyrimidine nucleotide binding [GO:0019103]; is a type of ribonucleotide binding [GO:0032553]